{
  "gene_symbol": "ATP8A2",
  "term_id": "GO:0005802",
  "term_label": "trans-Golgi network",
  "gene_name": "Phospholipid-transporting ATPase IB",
  "gene": "UniProtKB:Q9NTI2"
}